{
  "term_label": "Wnt receptor activity",
  "gene_name": "Frizzled-6",
  "gene": "UniProtKB:O60353",
  "gene_symbol": "FZD6",
  "term_id": "GO:0042813"
}